microtubule cytoskeleton attachment to nuclear envelope [GO:1990933] (biological process) Definition: A process in which the microtubule cytoskeleton is attached to the nuclear envelope. References: PMID:14655046, PMID:20507227 Relationships: is a type of microtubule cytoskeleton organization [GO:0000226]